{
  "term_label": "phototransduction",
  "gene_name": "Rhodopsin",
  "gene_symbol": "RHO",
  "term_id": "GO:0007602",
  "gene": "UniProtKB:P08100"
}